{
  "gene": "UniProtKB:A6NIJ9",
  "gene_symbol": "OR6C70",
  "gene_name": "Olfactory receptor 6C70",
  "term_label": "olfactory receptor activity",
  "term_id": "GO:0004984"
}